{
  "term_id": "GO:0045029",
  "gene": "UniProtKB:Q15077",
  "gene_symbol": "P2RY6",
  "gene_name": "P2Y purinoceptor 6",
  "term_label": "G protein-coupled UDP receptor activity"
}